{
  "gene_name": "Olfactory receptor 4K1",
  "term_id": "GO:0004984",
  "gene_symbol": "OR4K1",
  "term_label": "olfactory receptor activity",
  "gene": "UniProtKB:Q8NGD4"
}